{
  "gene_name": "Zinc finger protein 830",
  "gene_symbol": "ZNF830",
  "gene": "UniProtKB:Q96NB3",
  "term_id": "GO:0005634",
  "term_label": "nucleus"
}